{
  "gene_name": "Cell cycle regulator of non-homologous end joining",
  "gene_symbol": "CYREN",
  "term_label": "molecular adaptor activity",
  "gene": "UniProtKB:Q9BWK5",
  "term_id": "GO:0060090"
}